{
  "term_label": "ubiquitin protein ligase activity",
  "term_id": "GO:0061630",
  "gene": "UniProtKB:P22681",
  "gene_symbol": "CBL",
  "gene_name": "E3 ubiquitin-protein ligase CBL"
}